{
  "term_label": "cytosol",
  "term_id": "GO:0005829",
  "gene_symbol": "PSMA4",
  "gene_name": "Proteasome subunit alpha type-4",
  "gene": "UniProtKB:P25789"
}